sodium channel inhibitor activity [GO:0019871] (molecular function) Definition: Binds to and stops, prevents, or reduces the activity of a sodium channel. Relationships: is a type of ion channel inhibitor activity [GO:0008200]; is a type of sodium channel regulator activity [GO:0017080]; negatively regulates sodium channel activity [GO:0005272] Sources: GOC:mah